{
  "term_id": "GO:0030154",
  "term_label": "cell differentiation",
  "gene": "UniProtKB:Q5HYW2",
  "gene_name": "NHS-like protein 2",
  "gene_symbol": "NHSL2"
}